pinosylvin synthase activity [GO:0050198] (molecular function) Definition: Catalysis of the reaction: trans-cinnamoyl-CoA + 3 H+ + 3 malonyl-CoA = 4 CO2 + 4 CoA + pinosylvin. Sources: EC:2.3.1.146, RHEA:12552 Also known as: stilbene synthase activity, malonyl-CoA:cinnamoyl-CoA malonyltransferase (cyclizing), pine stilbene synthase activity Relationships: is a type of acyltransferase activity, transferring groups other than amino-acyl groups [GO:0016747]